{
  "term_id": "GO:0005737",
  "gene": "UniProtKB:Q9NP31",
  "gene_symbol": "SH2D2A",
  "gene_name": "SH2 domain-containing protein 2A",
  "term_label": "cytoplasm"
}